lipoprotein particle [GO:1990777] (cellular component) Definition: A spherical particle containing non-covalently associated proteins and lipids. Examples are plasma lipoprotein particles which transport lipids in the blood or lymph. Subtypes: plasma lipoprotein particle [GO:0034358] Relationships: is a type of protein-lipid complex [GO:0032994] Sources: GOC:vesicles